{
  "gene_name": "Transcription factor RFX4",
  "term_id": "GO:0005634",
  "term_label": "nucleus",
  "gene": "UniProtKB:Q33E94",
  "gene_symbol": "RFX4"
}